lipid homeostasis [GO:0055088] (biological process) Definition: Any process involved in the maintenance of an internal steady state of lipid within an organism or cell. Subtypes: brassinosteroid homeostasis [GO:0010268], GO:0010336, GO:0055089, GO:0055090, phospholipid homeostasis [GO:0055091], GO:0055092, GO:0090156, abscisic acid homeostasis [GO:1902265] Relationships: is a type of chemical homeostasis [GO:0048878] Sources: GOC:BHF, GOC:rl